{
  "gene_symbol": "TNR",
  "gene_name": "Tenascin-R",
  "term_label": "Unknown molecular function",
  "term_id": "UNKNOWN:0001",
  "gene": "UniProtKB:Q92752"
}